{
  "gene_name": "Apolipoprotein E",
  "term_id": "GO:0008203",
  "term_label": "cholesterol metabolic process",
  "gene_symbol": "APOE",
  "gene": "UniProtKB:P02649"
}